{
  "gene": "UniProtKB:Q7Z419",
  "term_id": "GO:0061630",
  "gene_symbol": "RNF144B",
  "gene_name": "E3 ubiquitin-protein ligase RNF144B",
  "term_label": "ubiquitin protein ligase activity"
}